{
  "gene_symbol": "CHDH",
  "term_label": "Unknown biological process",
  "gene_name": "Choline dehydrogenase, mitochondrial",
  "gene": "UniProtKB:Q8NE62",
  "term_id": "UNKNOWN:0002"
}